{
  "gene_symbol": "RAPGEF2",
  "term_label": "endocytic vesicle",
  "gene": "UniProtKB:Q9Y4G8",
  "gene_name": "Rap guanine nucleotide exchange factor 2",
  "term_id": "GO:0030139"
}